{
  "term_label": "Unknown cellular component",
  "gene_name": "Aminopeptidase RNPEPL1",
  "gene_symbol": "RNPEPL1",
  "gene": "UniProtKB:Q9HAU8",
  "term_id": "UNKNOWN:0003"
}